{
  "gene": "UniProtKB:Q9UPE1",
  "term_label": "protein serine/threonine kinase activity",
  "gene_symbol": "SRPK3",
  "term_id": "GO:0004674",
  "gene_name": "SRSF protein kinase 3"
}